{
  "gene_symbol": "PPARD",
  "term_id": "GO:0005634",
  "gene_name": "Peroxisome proliferator-activated receptor delta",
  "term_label": "nucleus",
  "gene": "UniProtKB:Q03181"
}